reactive oxygen species biosynthetic process [GO:1903409] (biological process) Also known as: reactive oxygen species anabolism, reactive oxygen species biosynthesis, reactive oxygen species formation, reactive oxygen species synthesis, ROS formation, ROS generation, reactive oxygen species generation Relationships: is a type of GO:0009058; is a type of reactive oxygen species metabolic process [GO:0072593] Regulation: RO_0002211 by regulation of reactive oxygen species biosynthetic process [GO:1903426]; negatively regulated by GO:1903427; positively regulated by positive regulation of reactive oxygen species biosynthetic process [GO:1903428] Subtypes: hypochlorous acid biosynthetic process [GO:0002149], hydrogen peroxide biosynthetic process [GO:0050665] Definition: The chemical reactions and pathways resulting in the formation of reactive oxygen species, any molecules or ions formed by the incomplete one-electron reduction of oxygen. References: PMID:24252804 Sources: GOC:PARL, GOC:TermGenie, GOC:bf, GO_REF:0000068